{
  "gene": "UniProtKB:Q99961",
  "term_label": "membrane",
  "gene_name": "Endophilin-A2",
  "gene_symbol": "SH3GL1",
  "term_id": "GO:0016020"
}